{
  "term_label": "cell fate commitment",
  "gene_name": "Protein Wnt-6",
  "gene": "UniProtKB:Q9Y6F9",
  "term_id": "GO:0045165",
  "gene_symbol": "WNT6"
}